{
  "term_label": "cytoplasm",
  "term_id": "GO:0005737",
  "gene_name": "RNA cytosine C(5)-methyltransferase NSUN2",
  "gene": "UniProtKB:Q08J23",
  "gene_symbol": "NSUN2"
}